{
  "term_label": "cellular response to estradiol stimulus",
  "gene": "UniProtKB:Q99527",
  "gene_name": "G-protein coupled estrogen receptor 1",
  "term_id": "GO:0071392",
  "gene_symbol": "GPER1"
}